negative regulation of circadian rhythm [GO:0042754] (biological process) Sources: GOC:go_curators Subtypes: negative regulation of circadian sleep/wake cycle, sleep [GO:0042321], negative regulation of locomotor rhythm [GO:1904060], GO:1904326 Also known as: down regulation of circadian rhythm, down-regulation of circadian rhythm, downregulation of circadian rhythm, inhibition of circadian rhythm Relationships: is_a GO:0042752; is a type of negative regulation of biological process [GO:0048519]; negatively regulates circadian rhythm [GO:0007623] Definition: Any process that stops, prevents, or reduces the frequency, rate or extent of a circadian rhythm behavior.